{
  "gene_symbol": "OPLAH",
  "gene": "UniProtKB:O14841",
  "term_id": "GO:0017168",
  "term_label": "5-oxoprolinase (ATP-hydrolyzing) activity",
  "gene_name": "5-oxoprolinase"
}